positive regulation of mast cell activation involved in immune response [GO:0033008] (biological process) Definition: Any process that activates or increases the frequency, rate, or extent of mast cell activation as part of an immune response. Sources: GOC:mah Also known as: positive regulation of mast cell activation during immune response Relationships: is a type of positive regulation of mast cell activation [GO:0033005]; is_a regulation of mast cell activation involved in immune response [GO:0033006]; is a type of positive regulation of immune response [GO:0050778]; positively regulates mast cell activation involved in immune response [GO:0002279]